{
  "gene_name": "Phosphatidylinositol N-acetylglucosaminyltransferase subunit Q",
  "gene_symbol": "PIGQ",
  "term_id": "GO:0005783",
  "gene": "UniProtKB:Q9BRB3",
  "term_label": "endoplasmic reticulum"
}